{
  "gene_name": "Neuropilin and tolloid-like protein 2",
  "gene_symbol": "NETO2",
  "term_id": "GO:0035255",
  "gene": "UniProtKB:Q8NC67",
  "term_label": "ionotropic glutamate receptor binding"
}